nuclear microtubule [GO:0005880] (cellular component) Definition: Any microtubule in the nucleus of a cell. Relationships: is a type of GO:0005874; is part of nucleus [GO:0005634] Sources: GOC:mah